{
  "gene_name": "Maestro heat-like repeat-containing protein family member 1",
  "term_id": "UNKNOWN:0001",
  "gene": "UniProtKB:Q8NDA8",
  "gene_symbol": "MROH1",
  "term_label": "Unknown molecular function"
}